gamma-catenin binding [GO:0045295] (molecular function) Relationships: is a type of protein binding [GO:0005515] Sources: GOC:bf Also known as: plakoglobin binding Definition: Binding to catenin complex gamma subunit.